{
  "term_label": "chloride channel activity",
  "gene_name": "Gamma-aminobutyric acid receptor subunit rho-1",
  "term_id": "GO:0005254",
  "gene": "UniProtKB:P24046",
  "gene_symbol": "GABRR1"
}